{
  "term_label": "phagophore assembly site",
  "gene_name": "Autophagy-related protein 13",
  "gene": "UniProtKB:O75143",
  "gene_symbol": "ATG13",
  "term_id": "GO:0000407"
}